{
  "gene_name": "B-cell receptor-associated protein 31",
  "gene_symbol": "BCAP31",
  "gene": "UniProtKB:P51572",
  "term_label": "endoplasmic reticulum to Golgi vesicle-mediated transport",
  "term_id": "GO:0006888"
}